{
  "gene": "UniProtKB:Q6UWM7",
  "term_label": "Unknown cellular component",
  "term_id": "UNKNOWN:0003",
  "gene_symbol": "LCTL",
  "gene_name": "Lactase-like protein"
}